{
  "gene": "UniProtKB:Q8IYB7",
  "gene_name": "DIS3-like exonuclease 2",
  "term_label": "miRNA catabolic process",
  "term_id": "GO:0010587",
  "gene_symbol": "DIS3L2"
}